{
  "term_label": "heterophilic cell-cell adhesion",
  "gene_name": "Pregnancy-specific beta-1-glycoprotein 11",
  "term_id": "GO:0007157",
  "gene": "UniProtKB:Q9UQ72",
  "gene_symbol": "PSG11"
}